{
  "gene_symbol": "GABRA3",
  "term_label": "dendrite membrane",
  "gene": "UniProtKB:P34903",
  "gene_name": "Gamma-aminobutyric acid receptor subunit alpha-3",
  "term_id": "GO:0032590"
}